regulation of cellular response to very-low-density lipoprotein particle stimulus [GO:1905890] (biological process) Also known as: regulation of cellular response to VLDL particle stimulus Relationships: is a type of GO:0048583; is a type of regulation of cellular process [GO:0050794]; regulates cellular response to very-low-density lipoprotein particle stimulus [GO:0090731] Definition: Any process that modulates the frequency, rate or extent of cellular response to very-low-density lipoprotein particle stimulus. Subtypes: GO:1905888, positive regulation of cellular response to very-low-density lipoprotein particle stimulus [GO:1905889] References: PMID:7592957 Sources: GOC:TermGenie, GOC:aruk, GOC:bc, GO_REF:0000058